{
  "gene_symbol": "AMOTL1",
  "gene": "UniProtKB:Q8IY63",
  "term_id": "GO:0035329",
  "term_label": "hippo signaling",
  "gene_name": "Angiomotin-like protein 1"
}